{
  "term_label": "secretory granule",
  "term_id": "GO:0030141",
  "gene_name": "Kallikrein-14",
  "gene_symbol": "KLK14",
  "gene": "UniProtKB:Q9P0G3"
}